{
  "gene_symbol": "COL4A2",
  "gene": "UniProtKB:P08572",
  "gene_name": "Collagen alpha-2(IV) chain",
  "term_label": "extracellular matrix",
  "term_id": "GO:0031012"
}